inositol phosphate kinase activity [GO:0180030] (molecular function) Subtypes: inositol-1,3,4,5,6-pentakisphosphate kinase activity [GO:0000827], inositol hexakisphosphate kinase activity [GO:0000828], diphosphoinositol pentakisphosphate kinase activity [GO:0000829], GO:0051765, inositol trisphosphate kinase activity [GO:0051766], inositol 5-diphosphate pentakisphosphate 5-kinase activity [GO:0052836], GO:0052839, inositol pentakisphosphate kinase activity [GO:0120517] Definition: Catalysis of the reaction: inositol phosphate + ATP = inositol phosphate + ADP. Relationships: is a type of kinase activity [GO:0016301] References: PMID:35536002